{
  "term_label": "dendrite self-avoidance",
  "gene_name": "Roundabout homolog 3",
  "gene": "UniProtKB:Q96MS0",
  "gene_symbol": "ROBO3",
  "term_id": "GO:0070593"
}